{
  "term_label": "manganese ion binding",
  "gene_symbol": "PCK2",
  "gene": "UniProtKB:Q16822",
  "gene_name": "Phosphoenolpyruvate carboxykinase [GTP], mitochondrial",
  "term_id": "GO:0030145"
}